effector-mediated activation of host programmed cell death by symbiont [GO:0034055] (biological process) Subtypes: effector-mediated activation of plant hypersensitive response by symbiont [GO:0080185] Sources: GOC:pamgo_curators Note: Note that this term is used to annotate gene products of the symbiont. Also known as: effector-mediated activation of programmed cell death in host, effector-mediated induction of programmed cell death in host, positive regulation by symbiont of host defense-related PCD, up regulation by symbiont of host defense-related programmed cell death, up-regulation by symbiont of host defense-related programmed cell death, upregulation by symbiont of host defense-related programmed cell death, activation by symbiont of host defense-related programmed cell death, enhancement by symbiont of host defense-related programmed cell death, stimulation by symbiont of host defense-related programmed cell death, positive regulation by symbiont of host defense-related programmed cell death Relationships: is a type of GO:0052042; is_a effector-mediated suppression of host innate immune response [GO:0140403] Definition: A symbiont process in which a molecule secreted by the symbiont activates a programmed cell death pathway in the host to suppress the host innate immune response. The host is defined as the larger of the organisms involved in a symbiotic interaction.